{
  "gene": "UniProtKB:Q96F86",
  "gene_name": "Enhancer of mRNA-decapping protein 3",
  "term_label": "mRNA binding",
  "gene_symbol": "EDC3",
  "term_id": "GO:0003729"
}